{
  "gene_name": "Syntaxin-binding protein 5-like",
  "term_id": "GO:0019905",
  "gene_symbol": "STXBP5L",
  "gene": "UniProtKB:Q9Y2K9",
  "term_label": "syntaxin binding"
}